{
  "gene_symbol": "MT3",
  "term_id": "GO:0071294",
  "gene": "UniProtKB:P25713",
  "term_label": "cellular response to zinc ion",
  "gene_name": "Metallothionein-3"
}